4-hydroxycoumarin biosynthetic process [GO:1901884] (biological process) Relationships: is a type of coumarin biosynthetic process [GO:0009805] References: PMID:19757094 Sources: GOC:TermGenie Definition: The chemical reactions and pathways resulting in the formation of 4-hydroxycoumarin. Also known as: 4-hydroxycoumarin anabolism, 4-hydroxycoumarin biosynthesis, 4-hydroxycoumarin formation, 4-hydroxycoumarin synthesis